{
  "gene": "UniProtKB:P37231",
  "gene_name": "Peroxisome proliferator-activated receptor gamma",
  "term_id": "GO:0045944",
  "gene_symbol": "PPARG",
  "term_label": "positive regulation of transcription by RNA polymerase II"
}